import into the mitochondrion [GO:0170036] (biological process) Relationships: is a type of GO:1990542 Sources: GOC:ew Subtypes: GO:0006850, GO:0140300, L-lysine transmembrane import into the mitochondrion [GO:0160256], isopentenyl pyrophosphate import into mitochondrion [GO:0170046], GO:1904983 Definition: The directed movement of substances from the cytosol into the mitochondrion.